{
  "gene": "UniProtKB:Q9NQT6",
  "term_label": "microvillus",
  "gene_name": "Fascin-3",
  "term_id": "GO:0005902",
  "gene_symbol": "FSCN3"
}